{
  "gene": "UniProtKB:Q6P5S7",
  "gene_name": "Ribonuclease kappa",
  "term_id": "UNKNOWN:0002",
  "gene_symbol": "RNASEK",
  "term_label": "Unknown biological process"
}